{
  "gene_name": "Proline-rich protein 15-like protein",
  "term_id": "UNKNOWN:0003",
  "gene_symbol": "PRR15L",
  "gene": "UniProtKB:Q9BU68",
  "term_label": "Unknown cellular component"
}